intramembranous bone growth [GO:0098867] (biological process) Relationships: is a type of bone growth [GO:0098868] Definition: The increase in size or mass of an intramembranous bone that contributes to the shaping of the bone. References: PMID:26399686